{
  "term_id": "GO:0039706",
  "term_label": "co-receptor binding",
  "gene": "UniProtKB:Q9UBP4",
  "gene_symbol": "DKK3",
  "gene_name": "Dickkopf-related protein 3"
}